anther wall tapetum morphogenesis [GO:0048655] (biological process) Sources: GOC:jid, GOC:sm, GOC:tb Also known as: tapetal layer morphogenesis, tapetum morphogenesis, differentiation of tapetal layer Definition: The process in which the anatomical structures of the anther wall tapetum are generated and organized. The anther wall tapetum is a layer of cells that provides a source of nutrition for the pollen grains as they mature. Relationships: is a type of GO:0003006; is a type of post-embryonic plant morphogenesis [GO:0090698]; is part of GO:0048654; is part of GO:0048658